phospholipid transporter activity [GO:0005548] (molecular function) Subtypes: phosphatidylcholine transporter activity [GO:0008525], aminophospholipid flippase activity [GO:0015247], GO:0017128, lysophospholipid:sodium symporter activity [GO:0051978], phosphatidylserine floppase activity [GO:0090556], GO:0120014, glycerophospholipid flippase activity [GO:0140333], GO:0140341, isopentenyl pyrophosphate transmembrane transporter activity [GO:0170045] Sources: GOC:ai, ISBN:0198506732 Definition: Enables the directed movement of phospholipids into, out of or within a cell, or between cells. Phospholipids are a class of lipids containing phosphoric acid as a mono- or diester. Relationships: is a type of lipid transporter activity [GO:0005319]; is part of phospholipid transport [GO:0015914]